positive regulation of lactose biosynthetic process [GO:1903536] (biological process) Definition: Any process that activates or increases the frequency, rate or extent of lactose biosynthetic process. References: PMID:12018418 Sources: GOC:TermGenie, GOC:mr, GO_REF:0000058 Also known as: positive regulation of lactose anabolism, positive regulation of lactose biosynthesis, positive regulation of lactose formation, positive regulation of lactose synthesis, up regulation of lactose anabolism, up regulation of lactose biosynthesis, up regulation of lactose biosynthetic process, up regulation of lactose formation, up regulation of lactose synthesis, up-regulation of lactose anabolism, up-regulation of lactose biosynthesis, up-regulation of lactose biosynthetic process, up-regulation of lactose formation, up-regulation of lactose synthesis, upregulation of lactose anabolism, upregulation of lactose biosynthesis, upregulation of lactose biosynthetic process, upregulation of lactose formation, upregulation of lactose synthesis, activation of lactose anabolism, activation of lactose biosynthesis, activation of lactose biosynthetic process, activation of lactose formation, activation of lactose synthesis Relationships: is a type of positive regulation of biosynthetic process [GO:0009891]; is a type of positive regulation of carbohydrate metabolic process [GO:0045913]; is a type of regulation of lactose biosynthetic process [GO:1903534]; positively regulates lactose biosynthetic process [GO:0005989]